3alpha-hydroxy-ent-sandaracopimardiene 7-beta-monooxygenase activity [GO:0102598] (molecular function) Definition: Catalysis of the reaction: ent-sandaracopimaradien-3-beta-ol + NADPH + H+ + O2 = oryzalexin D + NADP + H2O. Relationships: is_a oxidoreductase activity, acting on paired donors, with incorporation or reduction of molecular oxygen, NAD(P)H as one donor, and incorporation of one atom of oxygen [GO:0016709] Sources: EC:1.14.14.123, GOC:pz